N-methylcoclaurine 3'-monooxygenase activity [GO:0050593] (MF) Definition: Catalysis of the reaction: (S)-N-methylcoclaurine + H+ + NADPH + O2 = (S)-3'-hydroxy-N-methylcoclaurine + H2O + NADP+. Relationships: is a type of oxidoreductase activity, acting on paired donors, with incorporation or reduction of molecular oxygen, NAD(P)H as one donor, and incorporation of one atom of oxygen [GO:0016709] Also known as: N-methylcoclaurine 3'-hydroxylase activity, (S)-N-methylcoclaurine 3'-hydroxylase activity, (S)-N-methylcoclaurine,NADPH:oxygen oxidoreductase (3'-hydroxylating), cytochrome P450 80B1 activity Sources: EC:1.14.14.102, RHEA:16649